negative regulation of glutamate receptor signaling pathway [GO:1900450] (biological process) Definition: Any process that stops, prevents or reduces the frequency, rate or extent of glutamate receptor signaling pathway. Relationships: is a type of GO:0009968; is a type of GO:1900449; negatively regulates glutamate receptor signaling pathway [GO:0007215] Also known as: down regulation of glutamate receptor signaling pathway, down regulation of glutamate signaling pathway, down regulation of glutamate signalling pathway, down-regulation of glutamate receptor signaling pathway, down-regulation of glutamate signaling pathway, down-regulation of glutamate signalling pathway, downregulation of glutamate receptor signaling pathway, downregulation of glutamate signaling pathway, downregulation of glutamate signalling pathway, inhibition of glutamate signaling pathway, inhibition of glutamate signalling pathway, negative regulation of glutamate signaling pathway, negative regulation of glutamate signalling pathway, inhibition of glutamate receptor signaling pathway Sources: GOC:BHF, GOC:TermGenie